{
  "gene_name": "Putative zinc finger and SCAN domain-containing protein 5D",
  "gene": "UniProtKB:P0CG00",
  "gene_symbol": "ZSCAN5DP",
  "term_label": "regulation of transcription by RNA polymerase II",
  "term_id": "GO:0006357"
}